{
  "term_id": "GO:0003712",
  "gene": "UniProtKB:Q5U623",
  "gene_name": "Activating transcription factor 7-interacting protein 2",
  "gene_symbol": "ATF7IP2",
  "term_label": "transcription coregulator activity"
}